{
  "gene_symbol": "NXNL2",
  "gene": "UniProtKB:Q5VZ03",
  "term_label": "Unknown molecular function",
  "gene_name": "Nucleoredoxin-like protein 2",
  "term_id": "UNKNOWN:0001"
}